{
  "gene": "UniProtKB:A0A0G2JLJ8",
  "gene_name": "Immunoglobulin heavy diversity 5_OR15-5A (non-functional) (Fragment)",
  "gene_symbol": "IGHD5OR15-5B",
  "term_id": "UNKNOWN:0003",
  "term_label": "Unknown cellular component"
}